{
  "gene": "UniProtKB:Q9UN76",
  "term_label": "glycine import across plasma membrane",
  "term_id": "GO:1903804",
  "gene_symbol": "SLC6A14",
  "gene_name": "Sodium- and chloride-dependent neutral and basic amino acid transporter B(0+)"
}